negative regulation of positive thymic T cell selection [GO:1902233] (biological process) Definition: Any process that stops, prevents or reduces the frequency, rate or extent of positive thymic T cell selection. References: PMID:22080863 Sources: GOC:TermGenie Also known as: down regulation of positive thymic T cell selection, down regulation of positive thymic T lymphocyte selection, down regulation of positive thymic T-cell selection, down regulation of positive thymic T-lymphocyte selection, down-regulation of positive thymic T cell selection, down-regulation of positive thymic T lymphocyte selection, down-regulation of positive thymic T-cell selection, down-regulation of positive thymic T-lymphocyte selection, downregulation of positive thymic T cell selection, downregulation of positive thymic T lymphocyte selection, downregulation of positive thymic T-cell selection, downregulation of positive thymic T-lymphocyte selection, negative regulation of positive thymic T lymphocyte selection, negative regulation of positive thymic T-cell selection, negative regulation of positive thymic T-lymphocyte selection, inhibition of positive thymic T cell selection, inhibition of positive thymic T lymphocyte selection, inhibition of positive thymic T-cell selection, inhibition of positive thymic T-lymphocyte selection Relationships: is a type of GO:0033085; is a type of regulation of positive thymic T cell selection [GO:1902232]; negatively regulates positive thymic T cell selection [GO:0045059]